{
  "gene_name": "Very low-density lipoprotein receptor",
  "gene_symbol": "VLDLR",
  "term_label": "plasma membrane",
  "gene": "UniProtKB:P98155",
  "term_id": "GO:0005886"
}